UDP-xylosyltransferase activity [GO:0035252] (molecular function) Definition: Catalysis of the transfer of a xylosyl group from UDP-xylose to an acceptor molecule. Subtypes: protein xylosyltransferase activity [GO:0030158], dolichyl-phosphate D-xylosyltransferase activity [GO:0047283], flavonol-3-O-glycoside xylosyltransferase activity [GO:0047285], GO:0050404, GO:0050513, GO:0120053, xylosyl alpha-1,3-xylosyltransferase activity [GO:0140560], EGF-domain serine xylosyltransferase activity [GO:0140562], UDP-D-xylose:beta-D-glucoside alpha-1,3-D-xylosyltransferase activity [GO:0140563] References: PMID:30127001 Relationships: is a type of UDP-glycosyltransferase activity [GO:0008194]; is a type of GO:0042285